{
  "gene_name": "Heparan-sulfate 6-O-sulfotransferase 2",
  "gene_symbol": "HS6ST2",
  "term_label": "heparan sulfate 6-sulfotransferase activity",
  "term_id": "GO:0017095",
  "gene": "UniProtKB:Q96MM7"
}